{
  "term_label": "positive regulation of cytosolic calcium ion concentration",
  "gene": "UniProtKB:Q9P296",
  "term_id": "GO:0007204",
  "gene_name": "C5a anaphylatoxin chemotactic receptor 2",
  "gene_symbol": "C5AR2"
}